{
  "term_id": "GO:0000981",
  "gene": "UniProtKB:O95475",
  "gene_symbol": "SIX6",
  "gene_name": "Homeobox protein SIX6",
  "term_label": "DNA-binding transcription factor activity, RNA polymerase II-specific"
}